{
  "term_label": "Unknown molecular function",
  "gene": "UniProtKB:Q6NVV0",
  "gene_name": "Putative makorin-5",
  "gene_symbol": "MKRN9P",
  "term_id": "UNKNOWN:0001"
}